{
  "gene_name": "Prostate collagen triple helix protein",
  "term_label": "Unknown molecular function",
  "term_id": "UNKNOWN:0001",
  "gene": "UniProtKB:Q58A44",
  "gene_symbol": "PCOTH"
}